{
  "term_id": "UNKNOWN:0002",
  "gene_symbol": "AIRIM",
  "term_label": "Unknown biological process",
  "gene": "UniProtKB:Q9NX04",
  "gene_name": "AFG2-interacting ribosome maturation factor"
}